{
  "gene": "UniProtKB:Q14541",
  "term_id": "UNKNOWN:0003",
  "term_label": "Unknown cellular component",
  "gene_symbol": "HNF4G",
  "gene_name": "Hepatocyte nuclear factor 4-gamma"
}